{
  "term_label": "intrinsic apoptotic signaling pathway",
  "gene": "UniProtKB:P09912",
  "gene_name": "Interferon alpha-inducible protein 6",
  "term_id": "GO:0097193",
  "gene_symbol": "IFI6"
}